{
  "term_label": "chromatin",
  "gene_name": "Protein FAM47E",
  "gene_symbol": "FAM47E",
  "term_id": "GO:0000785",
  "gene": "UniProtKB:Q6ZV65"
}